{
  "term_label": "delayed rectifier potassium channel activity",
  "gene": "UniProtKB:P48547",
  "gene_name": "Potassium voltage-gated channel subfamily C member 1",
  "term_id": "GO:0005251",
  "gene_symbol": "KCNC1"
}